{
  "term_id": "GO:1990519",
  "gene": "UniProtKB:Q96CQ1",
  "gene_symbol": "SLC25A36",
  "term_label": "pyrimidine nucleotide import into mitochondrion",
  "gene_name": "Solute carrier family 25 member 36"
}